{
  "gene": "UniProtKB:Q7Z6I5",
  "gene_name": "Spermatogenesis-associated protein 12",
  "term_id": "UNKNOWN:0002",
  "gene_symbol": "SPATA12",
  "term_label": "Unknown biological process"
}